{
  "term_id": "GO:0043161",
  "gene_symbol": "PSMD2",
  "gene_name": "26S proteasome non-ATPase regulatory subunit 2",
  "term_label": "proteasome-mediated ubiquitin-dependent protein catabolic process",
  "gene": "UniProtKB:Q13200"
}